{
  "term_id": "GO:0030036",
  "gene_name": "PDZ and LIM domain protein 4",
  "term_label": "actin cytoskeleton organization",
  "gene_symbol": "PDLIM4",
  "gene": "UniProtKB:P50479"
}